{
  "gene_name": "Leucine--tRNA ligase, cytoplasmic",
  "term_id": "GO:0004823",
  "term_label": "leucine-tRNA ligase activity",
  "gene": "UniProtKB:Q9P2J5",
  "gene_symbol": "LARS1"
}